{
  "term_id": "UNKNOWN:0003",
  "gene": "UniProtKB:Q9BTF0",
  "gene_name": "THUMP domain-containing protein 2",
  "term_label": "Unknown cellular component",
  "gene_symbol": "THUMPD2"
}